SMC family protein binding [GO:0043221] (molecular function) Also known as: structural maintenance of chromosomes family protein binding Definition: Binding to a protein from the structural maintenance of chromosomes (SMC) family, a group of chromosomal ATPases with a role in mitotic chromosome organization. References: PMID:9640531 Sources: GOC:jl, GOC:vw, InterPro:IPR024704 Relationships: is_a protein binding [GO:0005515]